{
  "gene_name": "Selenide, water dikinase 2",
  "gene": "UniProtKB:Q99611",
  "term_label": "selenide, water dikinase activity",
  "term_id": "GO:0004756",
  "gene_symbol": "SEPHS2"
}